{
  "gene": "UniProtKB:P14868",
  "term_label": "aspartyl-tRNA aminoacylation",
  "term_id": "GO:0006422",
  "gene_symbol": "DARS1",
  "gene_name": "Aspartate--tRNA ligase, cytoplasmic"
}